{
  "term_id": "GO:0006816",
  "gene_symbol": "RAMP3",
  "term_label": "calcium ion transport",
  "gene_name": "Receptor activity-modifying protein 3",
  "gene": "UniProtKB:O60896"
}